eosinophil fate commitment [GO:0035854] (BP) Definition: The process in which the developmental fate of a cell becomes restricted such that it will develop into a eosinophil cell. A eosinophil is any of the immature or mature forms of a granular leukocyte with a nucleus that usually has two lobes connected by one or more slender threads of chromatin, and cytoplasm containing coarse, round granules that are uniform in size and which can be stained by the dye eosin. Sources: CL:0000771, GOC:BHF, GOC:vk Also known as: eosinophil cell fate commitment Relationships: is a type of cell fate commitment [GO:0045165]; is part of GO:0030222